{
  "term_id": "GO:0045277",
  "gene_symbol": "COX5A",
  "gene_name": "Cytochrome c oxidase subunit 5A, mitochondrial",
  "gene": "UniProtKB:P20674",
  "term_label": "respiratory chain complex IV"
}